{
  "term_id": "GO:0032981",
  "gene": "UniProtKB:Q9Y375",
  "term_label": "mitochondrial respiratory chain complex I assembly",
  "gene_name": "Complex I intermediate-associated protein 30, mitochondrial",
  "gene_symbol": "NDUFAF1"
}